{
  "term_label": "Unknown cellular component",
  "gene": "UniProtKB:Q8IZ02",
  "term_id": "UNKNOWN:0003",
  "gene_symbol": "LRRC34",
  "gene_name": "Leucine-rich repeat-containing protein 34"
}